{
  "gene_symbol": "SNX18",
  "term_id": "GO:0016197",
  "term_label": "endosomal transport",
  "gene_name": "Sorting nexin-18",
  "gene": "UniProtKB:Q96RF0"
}